{
  "gene": "UniProtKB:Q5JTC6",
  "gene_name": "APC membrane recruitment protein 1",
  "gene_symbol": "AMER1",
  "term_id": "GO:0060828",
  "term_label": "regulation of canonical Wnt signaling pathway"
}